{
  "gene_symbol": "TUT1",
  "gene": "UniProtKB:Q9H6E5",
  "gene_name": "Speckle targeted PIP5K1A-regulated poly(A) polymerase",
  "term_label": "poly(A) RNA polymerase activity",
  "term_id": "GO:1990817"
}